D-serine metabolic process [GO:0070178] (biological process) Subtypes: D-serine catabolic process [GO:0036088], D-serine biosynthetic process [GO:0070179] Also known as: D-serine metabolism Relationships: is a type of D-amino acid metabolic process [GO:0046416] Definition: The chemical reactions and pathways involving D-serine, the D-enantiomer of serine, i.e. (2R)-2-amino-3-hydroxypropanoic acid. Sources: CHEBI:16523, GOC:jsg, GOC:mah